{
  "term_label": "acetylcholine receptor inhibitor activity",
  "gene_name": "Secreted Ly-6_uPAR domain-containing protein 2",
  "term_id": "GO:0030550",
  "gene": "UniProtKB:P0DP57",
  "gene_symbol": "SLURP2"
}